{
  "term_id": "UNKNOWN:0003",
  "gene_symbol": "PYURF",
  "term_label": "Unknown cellular component",
  "gene": "UniProtKB:Q96I23",
  "gene_name": "Protein preY, mitochondrial"
}